midbrain-hindbrain boundary development [GO:0030917] (biological process) Definition: The process whose specific outcome is the progression of the midbrain-hindbrain boundary over time, from its formation to the mature structure. The midbrain-hindbrain domain of the embryonic brain is comprised of the mesencephalic vesicle and the first rhombencephalic vesicle at early somitogenesis stages. Sources: GOC:dgh Also known as: MHB development, isthmic organizer development, isthmomesencephalic boundary development, isthmus development, midbrain-hindbrain orgainizer development Relationships: is a type of anatomical structure development [GO:0048856]; is part of GO:0007420; is part of GO:0021903